dendritic microtubule [GO:1901588] (cellular component) Sources: GOC:TermGenie, NIF_Subcellular:sao110773650 Also known as: microtubule of dendrite, microtubulus of dendrite Relationships: is a type of microtubule [GO:0005874]; is part of dendrite [GO:0030425] Definition: Any microtubule in a dendrite, a neuron projection.